{
  "term_id": "GO:0005737",
  "gene": "UniProtKB:Q9UBS9",
  "gene_symbol": "SUCO",
  "gene_name": "SUN domain-containing ossification factor",
  "term_label": "cytoplasm"
}